positive regulation of anterograde dense core granule transport [GO:1901953] (biological process) References: PMID:23358451 Sources: GOC:TermGenie, GOC:kmv Also known as: up regulation of anterograde dense core granule transport, up-regulation of anterograde dense core granule transport, upregulation of anterograde dense core granule transport, activation of anterograde dense core granule transport Definition: Any process that activates or increases the frequency, rate or extent of anterograde dense core granule transport. Relationships: is a type of positive regulation of vesicle transport along microtubule [GO:1901610]; is_a regulation of anterograde dense core granule transport [GO:1901951]; is a type of positive regulation of dense core granule transport [GO:1904811]; positively regulates GO:1990048